phenylalanine racemase (ATP-hydrolyzing) activity [GO:0047462] (molecular function) Definition: Catalysis of the reaction: L-phenylalanine + ATP + H2O = D-phenylalanine + AMP + diphosphate + 2 H+. Sources: EC:5.1.1.11, RHEA:20201 Relationships: is a type of amino-acid racemase activity [GO:0047661] Also known as: phenylalanine racemase (ATP-hydrolysing), gramicidin S synthetase I, phenylalanine racemase (adenosine triphosphate-hydrolysing), phenylalanine racemase activity